{
  "gene_name": "Translin-associated protein X",
  "gene": "UniProtKB:Q99598",
  "gene_symbol": "TSNAX",
  "term_id": "GO:0005634",
  "term_label": "nucleus"
}